primary alcohol biosynthetic process [GO:0034309] (biological process) Also known as: monohydric alcohol biosynthetic process, primary alcohol anabolism, primary alcohol biosynthesis, primary alcohol formation, primary alcohol synthesis Sources: GOC:mah Subtypes: ethanol biosynthetic process [GO:0006115], GO:0006715, thiamine biosynthetic process [GO:0009228], aldosterone biosynthetic process [GO:0032342], phytol biosynthetic process [GO:0033520], GO:0034651, chrysobactin biosynthetic process [GO:0042858], methanol biosynthetic process [GO:0046169], octanol biosynthetic process [GO:0046171], glycolate biosynthetic process [GO:0046295], GO:0046335, 1-butanol biosynthetic process [GO:0071271], vomitoxin biosynthetic process [GO:0106110], isobutanol biosynthetic process [GO:1901961], (+)-lariciresinol biosynthetic process [GO:1902132], aromatic primary alcohol biosynthetic process [GO:1902655], geraniol biosynthetic process [GO:1903448], GO:2001317 Relationships: is a type of primary alcohol metabolic process [GO:0034308]; is a type of GO:0046165 Definition: The chemical reactions and pathways resulting in the formation of primary alcohols. A primary alcohol is any alcohol in which a hydroxy group, -OH, is attached to a saturated carbon atom which has either three hydrogen atoms attached to it or only one other carbon atom and two hydrogen atoms attached to it.